{
  "term_id": "GO:0045121",
  "gene_symbol": "CBLB",
  "term_label": "membrane raft",
  "gene": "UniProtKB:Q13191",
  "gene_name": "E3 ubiquitin-protein ligase CBL-B"
}